{
  "gene_symbol": "NLRP14",
  "term_label": "regulation of inflammatory response",
  "gene": "UniProtKB:Q86W24",
  "term_id": "GO:0050727",
  "gene_name": "NACHT, LRR and PYD domains-containing protein 14"
}